ERMES complex [GO:0032865] (cellular component) Definition: A protein complex that links the endoplasmic reticulum with mitochondria and may have a role in promoting exchange of calcium and phospholipids between the two organelles. References: PMID:19556461, PMID:29279306 Sources: GOC:mcc Also known as: ER-mitochondria encounter structure, MMM1 complex, Mdm10/Mdm12/Mmm1 complex, mitochore Relationships: is a type of GO:0098799; is a type of endoplasmic reticulum protein-containing complex [GO:0140534]; is part of GO:0044233